{
  "gene_symbol": "POLR3H",
  "gene": "UniProtKB:Q9Y535",
  "term_label": "transcription initiation at RNA polymerase III promoter",
  "term_id": "GO:0006384",
  "gene_name": "DNA-directed RNA polymerase III subunit RPC8"
}